{
  "term_id": "GO:0003714",
  "gene_symbol": "IRF2BP1",
  "gene": "UniProtKB:Q8IU81",
  "term_label": "transcription corepressor activity",
  "gene_name": "Interferon regulatory factor 2-binding protein 1"
}